axonemal central pair projection [GO:1990718] (cellular component) References: PMID:21586547, PMID:9295136 Sources: GOC:cilia Definition: Part of the 9+2 axoneme, that occurs in most motile cilia, consisting of the projections off of the central pair of single microtubules. Relationships: is a type of cellular anatomical structure [GO:0110165]; is part of axonemal central apparatus [GO:1990716]